{
  "gene_symbol": "EPAS1",
  "gene_name": "Endothelial PAS domain-containing protein 1",
  "term_label": "erythrocyte differentiation",
  "term_id": "GO:0030218",
  "gene": "UniProtKB:Q99814"
}